{
  "gene_name": "Uncharacterized protein C15orf62, mitochondrial",
  "gene_symbol": "C15orf62",
  "term_id": "GO:0005737",
  "term_label": "cytoplasm",
  "gene": "UniProtKB:A8K5M9"
}